{
  "gene": "UniProtKB:Q5TB80",
  "gene_name": "Centrosomal protein of 162 kDa",
  "term_label": "centriolar satellite",
  "term_id": "GO:0034451",
  "gene_symbol": "CEP162"
}